{
  "gene_symbol": "IP6K1",
  "term_label": "cytoplasm",
  "gene_name": "Inositol hexakisphosphate kinase 1",
  "term_id": "GO:0005737",
  "gene": "UniProtKB:Q92551"
}